{
  "gene_name": "Mannosyl-oligosaccharide 1,2-alpha-mannosidase IA",
  "term_label": "mannosyl-oligosaccharide 1,2-alpha-mannosidase activity",
  "term_id": "GO:0004571",
  "gene_symbol": "MAN1A1",
  "gene": "UniProtKB:P33908"
}